{
  "gene": "UniProtKB:P19484",
  "term_id": "GO:0005634",
  "term_label": "nucleus",
  "gene_symbol": "TFEB",
  "gene_name": "Transcription factor EB"
}